cellular response to low-density lipoprotein particle stimulus [GO:0071404] (biological process) Definition: Any process that results in a change in state or activity of a cell (in terms of movement, secretion, enzyme production, gene expression, etc.) as a result of a low-density lipoprotein particle stimulus. Relationships: is a type of response to lipoprotein particle [GO:0055094]; is a type of cellular response to lipoprotein particle stimulus [GO:0071402] Also known as: response to low density lipoprotein particle, response to low-density lipoprotein particle, response to low-density lipoprotein particle stimulus Subtypes: cellular response to oxidised low-density lipoprotein particle stimulus [GO:0140052] Sources: GOC:mah